histone H1 reader activity [GO:0140128] (molecular function) References: PMID:17540172 Relationships: is a type of histone reader activity [GO:0140566] Definition: A histone reader that specifically binds either to an unmodified histone H1 or a form modified by a post-translational modification on a specific residue. The most common PTMs on histones are methylation, acetylation and phosphorylation. Subtypes: histone H1K26me1 reader activity [GO:0160267], GO:0160268